apical pole of neuron [GO:0044225] (cellular component) Sources: NIF_Subcellular:sao1186862860 Relationships: is a type of cell pole [GO:0060187]; is part of GO:0043025 Definition: Portion of a neuron cell soma closest to the point where the apical dendrite emerges.